{
  "term_id": "GO:0043235",
  "gene_name": "Proto-oncogene tyrosine-protein kinase ROS",
  "gene": "UniProtKB:P08922",
  "term_label": "receptor complex",
  "gene_symbol": "ROS1"
}